{
  "term_label": "DNA-binding transcription factor activity, RNA polymerase II-specific",
  "gene": "UniProtKB:Q13106",
  "gene_symbol": "ZNF154",
  "gene_name": "Zinc finger protein 154",
  "term_id": "GO:0000981"
}